{
  "gene_symbol": "PPIL3",
  "gene": "UniProtKB:Q9H2H8",
  "term_label": "Unknown biological process",
  "term_id": "UNKNOWN:0002",
  "gene_name": "Peptidyl-prolyl cis-trans isomerase-like 3"
}